regulation of vegetative phase change [GO:0010321] (biological process) Definition: Any process that modulates the frequency, rate or extent of vegetative phase change. Vegetative phase change is the set of post-embryonic processes involved in the transition of a plant from a juvenile phase of vegetative development to an adult phase of vegetative development. Sources: GOC:tair_curators Relationships: is a type of regulation of post-embryonic development [GO:0048580]; regulates vegetative phase change [GO:0010050]